{
  "gene_symbol": "SEMA4D",
  "gene": "UniProtKB:Q92854",
  "term_label": "semaphorin-plexin signaling pathway",
  "gene_name": "Semaphorin-4D",
  "term_id": "GO:0071526"
}